{
  "term_id": "GO:0071028",
  "gene": "UniProtKB:Q15024",
  "gene_symbol": "EXOSC7",
  "gene_name": "Exosome complex component RRP42",
  "term_label": "nuclear mRNA surveillance"
}